{
  "gene_symbol": "RAB11FIP3",
  "gene": "UniProtKB:O75154",
  "term_id": "GO:0032154",
  "term_label": "cleavage furrow",
  "gene_name": "Rab11 family-interacting protein 3"
}